{
  "gene": "UniProtKB:Q7Z3K6",
  "term_id": "GO:0000122",
  "gene_name": "Mesoderm induction early response protein 3",
  "gene_symbol": "MIER3",
  "term_label": "negative regulation of transcription by RNA polymerase II"
}